{
  "term_label": "immunoglobulin mediated immune response",
  "term_id": "GO:0016064",
  "gene_symbol": "IGHV3-43",
  "gene": "UniProtKB:A0A0B4J1X8",
  "gene_name": "Immunoglobulin heavy variable 3-43"
}